{
  "gene_name": "Choline-phosphate cytidylyltransferase A",
  "gene_symbol": "PCYT1A",
  "term_label": "endoplasmic reticulum",
  "term_id": "GO:0005783",
  "gene": "UniProtKB:P49585"
}